{
  "term_label": "negative regulation of Notch signaling pathway",
  "gene": "UniProtKB:Q9NWT6",
  "term_id": "GO:0045746",
  "gene_name": "Hypoxia-inducible factor 1-alpha inhibitor",
  "gene_symbol": "HIF1AN"
}